{
  "gene_name": "Multiple epidermal growth factor-like domains protein 11",
  "gene_symbol": "MEGF11",
  "gene": "UniProtKB:A6BM72",
  "term_id": "GO:0005604",
  "term_label": "basement membrane"
}